{
  "term_id": "GO:0008017",
  "term_label": "microtubule binding",
  "gene_name": "Kinesin-like protein KIF16B",
  "gene_symbol": "KIF16B",
  "gene": "UniProtKB:Q96L93"
}